{
  "term_label": "Unknown cellular component",
  "term_id": "UNKNOWN:0003",
  "gene_name": "Uncharacterized protein FLJ46757",
  "gene_symbol": "Q6ZR03",
  "gene": "UniProtKB:Q6ZR03"
}